regulation of fever generation by regulation of prostaglandin biosynthesis [GO:0071809] (biological process) Sources: GOC:BHF, GOC:dph, GOC:mah Definition: Any process that modulates the rate or extent of fever generation via regulation of the frequency, rate or extent of the chemical reactions and pathways resulting in the formation of prostaglandin. Relationships: is a type of GO:0031392; is a type of regulation of fever generation [GO:0031620]; regulates regulation of fever generation by prostaglandin biosynthetic process [GO:0100008]